{
  "gene": "UniProtKB:P28329",
  "term_id": "GO:0005737",
  "gene_name": "Choline O-acetyltransferase",
  "gene_symbol": "CHAT",
  "term_label": "cytoplasm"
}